{
  "term_label": "Unknown biological process",
  "term_id": "UNKNOWN:0002",
  "gene_symbol": "ACP7",
  "gene": "UniProtKB:Q6ZNF0",
  "gene_name": "Acid phosphatase type 7"
}